{
  "term_label": "regulation of transcription by RNA polymerase II",
  "gene": "UniProtKB:P17041",
  "gene_name": "Zinc finger protein 32",
  "gene_symbol": "ZNF32",
  "term_id": "GO:0006357"
}